voltage-gated calcium channel complex assembly [GO:0070978] (biological process) Sources: GOC:mh Relationships: is a type of GO:0065003 Definition: Cellular protein complex assembly that results in the formation of a voltage-gated calcium channel complex.